substance K receptor binding [GO:0031837] (molecular function) Also known as: neurokinin-A receptor binding, substance K receptor ligand Relationships: is_a neurokinin receptor binding [GO:0031834] Sources: GOC:mah, GOC:nln Definition: Binding to a substance K receptor.